{
  "gene_name": "Protein Wnt-9a",
  "term_label": "neuron differentiation",
  "term_id": "GO:0030182",
  "gene_symbol": "WNT9A",
  "gene": "UniProtKB:O14904"
}